{
  "gene": "UniProtKB:Q68CP9",
  "gene_name": "AT-rich interactive domain-containing protein 2",
  "gene_symbol": "ARID2",
  "term_id": "UNKNOWN:0002",
  "term_label": "Unknown biological process"
}